N-acetylgalactosamine-6-sulfatase activity [GO:0043890] (MF) Relationships: is_a sulfuric ester hydrolase activity [GO:0008484] Sources: EC:3.1.6.4 Also known as: chondroitin sulfatase, chondroitinase, chondroitinsulfatase, N-acetyl-D-galactosamine-6-sulfate 6-sulfohydrolase activity, N-acetylgalactosamine 6-sulfatase activity, N-acetylgalactosamine-6-sulfate sulfatase activity, acetylgalactosamine 6-sulfatase activity, galactose-6-sulfate sulfatase activity Definition: Catalysis of the hydrolysis of the 6-sulfate groups of the N-acetyl-D-galactosamine 6-sulfate units of chondroitin sulfate and of the D-galactose 6-sulfate units of keratan sulfate.